regulation of chemokinesis [GO:1904365] (biological process) Definition: Any process that modulates the frequency, rate or extent of chemokinesis. Relationships: is a type of regulation of response to external stimulus [GO:0032101]; regulates chemokinesis [GO:0042466] References: PMID:8679543 Sources: GOC:TermGenie, GO_REF:0000058 Subtypes: GO:1904366, positive regulation of chemokinesis [GO:1904367]